{
  "term_id": "GO:0005886",
  "gene_name": "Laminin subunit alpha-2",
  "gene": "UniProtKB:P24043",
  "term_label": "plasma membrane",
  "gene_symbol": "LAMA2"
}